L-arabinose transmembrane transporter activity [GO:0015147] (molecular function) Relationships: is a type of GO:0042900 Definition: Enables the transfer of L-arabinose from one side of a membrane to the other. Arabinose occurs free, for example in the heartwood of many conifers and in the combined states, in both furanose and pyranose forms, as a constituent of various plant hemicelluloses, bacterial polysaccharides, etc. Subtypes: ABC-type L-arabinose transporter activity [GO:0015612] Sources: GOC:mtg_transport, ISBN:0198506732, ISBN:0815340729 Also known as: L-arabinose/beta-D-thiogalactopyranoside:hydrogen antiporter activity